{
  "gene_symbol": "CCL11",
  "term_label": "CCR chemokine receptor binding",
  "gene_name": "Eotaxin",
  "term_id": "GO:0048020",
  "gene": "UniProtKB:P51671"
}